{
  "term_id": "UNKNOWN:0001",
  "gene_symbol": "CXorf49B",
  "gene_name": "Uncharacterized protein CXorf49",
  "gene": "UniProtKB:A8MYA2",
  "term_label": "Unknown molecular function"
}